double-stranded methylated DNA binding [GO:0010385] (molecular function) Definition: Binding to double-stranded methylated DNA. Methylation of cytosine or adenine in DNA is an important mechanism for establishing stable heritable epigenetic marks. Relationships: is a type of double-stranded DNA binding [GO:0003690] References: PMID:17242155 Sources: GOC:imk